peripheral tolerance induction to nonself antigen [GO:0002464] (biological process) Sources: GOC:jal, ISBN:0781735149 Definition: Tolerance induction to nonself antigens in the periphery. Relationships: is a type of tolerance induction to nonself antigen [GO:0002462]; is a type of peripheral tolerance induction [GO:0002465]